{
  "term_label": "cytoplasm",
  "gene_symbol": "OPA1",
  "gene_name": "Dynamin-like 120 kDa protein, mitochondrial",
  "gene": "UniProtKB:O60313",
  "term_id": "GO:0005737"
}